negative regulation of cytoplasmic mRNA processing body assembly [GO:0010607] (biological process) Definition: Any process that decreases the rate, frequency, or extent of the aggregation, arrangement and bonding together of proteins and RNA molecules to form a cytoplasmic mRNA processing body. Relationships: is a type of regulation of cytoplasmic mRNA processing body assembly [GO:0010603]; is a type of negative regulation of organelle assembly [GO:1902116]; negatively regulates P-body assembly [GO:0033962] Sources: GOC:dph, GOC:krc, GOC:tb